{
  "gene_name": "Calcium-binding protein 8",
  "gene_symbol": "CALN1",
  "gene": "UniProtKB:Q9BXU9",
  "term_id": "UNKNOWN:0002",
  "term_label": "Unknown biological process"
}